{
  "gene_name": "Homeodomain-interacting protein kinase 4",
  "gene_symbol": "HIPK4",
  "term_label": "nucleus",
  "gene": "UniProtKB:Q8NE63",
  "term_id": "GO:0005634"
}